regulation of renal output by angiotensin [GO:0002019] (biological process) Also known as: angiotensin mediated regulation of renal output, angiotensin-mediated regulation of renal output, angiotensin mediated control of renal output Subtypes: negative regulation of renal output by angiotensin [GO:0003083] Sources: GOC:dph, GOC:mtg_cardio, GOC:tb, ISBN:0721643949 Definition: The process in which angiotensin directly modulates the rate of urine output by the kidney. Relationships: is_a regulation of blood volume by renin-angiotensin [GO:0002016]